{
  "term_id": "GO:0000981",
  "gene_name": "Transcriptional repressor protein YY1",
  "term_label": "DNA-binding transcription factor activity, RNA polymerase II-specific",
  "gene": "UniProtKB:P25490",
  "gene_symbol": "YY1"
}